{
  "gene": "UniProtKB:Q02641",
  "gene_name": "Voltage-dependent L-type calcium channel subunit beta-1",
  "term_id": "GO:0007268",
  "gene_symbol": "CACNB1",
  "term_label": "chemical synaptic transmission"
}